{
  "term_id": "GO:0004222",
  "term_label": "metalloendopeptidase activity",
  "gene_symbol": "MME",
  "gene": "UniProtKB:P08473",
  "gene_name": "Neprilysin"
}